HFE-transferrin receptor complex [GO:1990712] (cellular component) Definition: A protein complex containing at least HFE and a transferrin receptor (either TFR1/TFRC or TFR2), proposed to play a role in the sensing of transferrin-bound Fe (Fe2-Tf) on the plasma membrane to regulate hepcidin transcription. Relationships: is a type of plasma membrane signaling receptor complex [GO:0098802] References: PMID:25147378 Sources: GOC:BHF, GOC:kom